neural crest cell fate determination [GO:0014035] (biological process) Definition: The process in which a cell becomes capable of differentiating autonomously into a neural crest cell regardless of its environment; upon determination, the cell fate cannot be reversed. Sources: GOC:dh, GOC:ef Relationships: is a type of stem cell fate determination [GO:0048867]; is part of GO:0014034